{
  "term_id": "UNKNOWN:0002",
  "term_label": "Unknown biological process",
  "gene": "UniProtKB:Q64LD2",
  "gene_symbol": "WDR25",
  "gene_name": "WD repeat-containing protein 25"
}